{
  "gene": "UniProtKB:Q9NQ36",
  "gene_name": "Signal peptide, CUB and EGF-like domain-containing protein 2",
  "term_id": "GO:0007165",
  "gene_symbol": "SCUBE2",
  "term_label": "signal transduction"
}